{
  "gene_symbol": "LDB3",
  "term_label": "actin binding",
  "gene": "UniProtKB:O75112",
  "term_id": "GO:0003779",
  "gene_name": "LIM domain-binding protein 3"
}